{
  "gene_symbol": "PNLDC1",
  "term_id": "GO:0003723",
  "gene_name": "Poly(A)-specific ribonuclease PNLDC1",
  "gene": "UniProtKB:Q8NA58",
  "term_label": "RNA binding"
}